{
  "term_id": "GO:0007155",
  "gene": "UniProtKB:Q9UN75",
  "gene_symbol": "PCDHA12",
  "term_label": "cell adhesion",
  "gene_name": "Protocadherin alpha-12"
}